phosphoenolpyruvate-dependent mannosylglycerate phosphotransferase system [GO:0051476] (biological process) Relationships: is a type of phosphoenolpyruvate-dependent sugar phosphotransferase system [GO:0009401]; is a type of glycoside transport [GO:1901656]; is a type of GO:1905039 Definition: A phosphoenolpyruvate-dependent sugar phosphotransferase transport specific for mammosylglycerate. Also known as: mannosylglycerate transport References: PMID:368051